primary ovarian follicle growth [GO:0001545] (biological process) Subtypes: primary ovarian follicle growth involved in double layer follicle stage [GO:0043929], primary ovarian follicle growth involved in primary follicle stage [GO:0043930] Relationships: is a type of GO:0022602; is_a developmental growth [GO:0048589]; is part of GO:0001541 Sources: GOC:mtg_mpo, https://www.ncbi.nlm.nih.gov/books/NBK279054/ Definition: Increase in size of primary follicles including oocyte growth and granulosa and/or theca cell proliferation until more than one layer of granulosa cells is present (preantral follicle).